{
  "term_id": "GO:0006955",
  "gene_name": "Immunoglobulin kappa variable 1-12",
  "term_label": "immune response",
  "gene": "UniProtKB:A0A0C4DH73",
  "gene_symbol": "IGKV1-12"
}